{
  "gene": "UniProtKB:Q9H1B7",
  "term_label": "Unknown cellular component",
  "term_id": "UNKNOWN:0003",
  "gene_symbol": "IRF2BPL",
  "gene_name": "Probable E3 ubiquitin-protein ligase IRF2BPL"
}